{
  "term_id": "UNKNOWN:0002",
  "gene_symbol": "MAD2L1BP",
  "term_label": "Unknown biological process",
  "gene_name": "MAD2L1-binding protein",
  "gene": "UniProtKB:Q15013"
}